{
  "term_id": "GO:0000149",
  "gene_name": "Syntaxin-16",
  "gene_symbol": "STX16",
  "gene": "UniProtKB:O14662",
  "term_label": "SNARE binding"
}